mitochondrion-endoplasmic reticulum membrane tether activity [GO:0140474] (molecular function) Relationships: is a type of endoplasmic reticulum-organelle membrane tether activity [GO:0170009] Definition: The binding activity of a molecule that brings together a mitochondrion and an ER membrane either via membrane lipid binding or by interacting with a mitochondrial outer membrane protein, to establish or maintain the localization of the mitochondrion. References: PMID:19556461, PMID:27875684 Also known as: ER-mitochondrion membrane adaptor activity, ER-mitochondrion membrane tether activity, endoplasmic reticulum-mitochondrion membrane adaptor activity, endoplasmic reticulum-mitochondrion membrane tether activity, mitochondrion-ER membrane adaptor activity, mitochondrion-ER membrane tether activity, mitochondrion-endoplasmic reticulum membrane adaptor activity